regulation of cordyol C biosynthetic process [GO:1900861] (BP) Definition: Any process that modulates the frequency, rate or extent of cordyol C biosynthetic process. Sources: GOC:TermGenie, GOC:di Relationships: is a type of regulation of secondary metabolite biosynthetic process [GO:1900376]; regulates cordyol C biosynthetic process [GO:1900799] Subtypes: GO:1900862, positive regulation of cordyol C biosynthetic process [GO:1900863]